{
  "gene_name": "Mitochondrial fission regulator 1-like",
  "gene_symbol": "MTFR1L",
  "term_id": "GO:0000266",
  "gene": "UniProtKB:Q9H019",
  "term_label": "mitochondrial fission"
}